{
  "gene_symbol": "SYNJ1",
  "gene": "UniProtKB:O43426",
  "term_id": "GO:0005737",
  "gene_name": "Synaptojanin-1",
  "term_label": "cytoplasm"
}